{
  "gene": "UniProtKB:P01730",
  "term_id": "GO:0005102",
  "term_label": "signaling receptor binding",
  "gene_symbol": "CD4",
  "gene_name": "T-cell surface glycoprotein CD4"
}